{
  "gene": "UniProtKB:O00762",
  "term_id": "GO:0031145",
  "gene_symbol": "UBE2C",
  "term_label": "anaphase-promoting complex-dependent catabolic process",
  "gene_name": "Ubiquitin-conjugating enzyme E2 C"
}